{
  "gene": "UniProtKB:P31151",
  "term_id": "GO:0005737",
  "gene_symbol": "S100A7",
  "gene_name": "Protein S100-A7",
  "term_label": "cytoplasm"
}